conjugation with mutual genetic exchange [GO:0000748] (biological process) Relationships: is a type of sexual reproduction [GO:0019953] References: PMID:22444146 Sources: GOC:elh Also known as: conjugation without cellular fusion Definition: A conjugation process that results in the mutual exchange and union of only genetic information between compatible mating types. Conjugation without cellular fusion requires direct cellular contact between the organisms without plasma membrane fusion. The organisms involved in conjugation without cellular fusion separate after nuclear exchange. Regulation: RO_0002211 by GO:0000756